L-methionine secondary active transmembrane transporter activity [GO:0000102] (molecular function) Definition: Enables the transfer of L-methionine from one side of a membrane to the other, up its concentration gradient. The transporter binds the solute and undergoes a series of conformational changes. Transport works equally well in either direction and is driven by a chemiosmotic source of energy. Secondary active transporters include symporters and antiporters. Relationships: is a type of neutral L-amino acid secondary active transmembrane transporter activity [GO:0005294]; is a type of L-methionine transmembrane transporter activity [GO:0015191] Sources: GOC:mtg_transport Also known as: L-methionine porter activity